{
  "term_id": "GO:0007224",
  "term_label": "smoothened signaling pathway",
  "gene": "UniProtKB:Q9H2X6",
  "gene_symbol": "HIPK2",
  "gene_name": "Homeodomain-interacting protein kinase 2"
}